{
  "gene_symbol": "RFC4",
  "gene": "UniProtKB:P35249",
  "gene_name": "Replication factor C subunit 4",
  "term_id": "GO:0006281",
  "term_label": "DNA repair"
}